{
  "term_id": "GO:0006357",
  "gene_name": "Zinc finger protein 57",
  "gene": "UniProtKB:Q68EA5",
  "term_label": "regulation of transcription by RNA polymerase II",
  "gene_symbol": "ZNF57"
}